{
  "gene": "UniProtKB:Q6IF42",
  "term_label": "detection of chemical stimulus involved in sensory perception of smell",
  "term_id": "GO:0050911",
  "gene_name": "Olfactory receptor 2A2",
  "gene_symbol": "OR2A2"
}